fibroblast proliferation [GO:0048144] (biological process) Regulation: regulated by regulation of fibroblast proliferation [GO:0048145]; positively regulated by positive regulation of fibroblast proliferation [GO:0048146]; negatively regulated by negative regulation of fibroblast proliferation [GO:0048147] Definition: The multiplication or reproduction of fibroblast cells, resulting in the expansion of the fibroblast population. Relationships: is a type of cell population proliferation [GO:0008283] Sources: GOC:jid Subtypes: fibroblast proliferation involved in heart morphogenesis [GO:0061385], GO:0072343, hepatic stellate cell proliferation [GO:1990922]